{
  "term_id": "GO:0015629",
  "term_label": "actin cytoskeleton",
  "gene_name": "Unconventional myosin-Ig",
  "gene_symbol": "MYO1G",
  "gene": "UniProtKB:B0I1T2"
}